{
  "gene_name": "Immunoglobulin heavy diversity 6-19 (Fragment)",
  "gene_symbol": "IGHD6-19",
  "term_label": "Unknown biological process",
  "term_id": "UNKNOWN:0002",
  "gene": "UniProtKB:A0A1Y8EKQ5"
}